{
  "term_label": "Unknown biological process",
  "gene": "UniProtKB:Q6Q6R5",
  "gene_symbol": "CRIP3",
  "gene_name": "Cysteine-rich protein 3",
  "term_id": "UNKNOWN:0002"
}